{
  "gene_symbol": "TNPO1",
  "gene": "UniProtKB:Q92973",
  "term_id": "GO:0006606",
  "term_label": "protein import into nucleus",
  "gene_name": "Transportin-1"
}